{
  "gene_name": "Signal transducer and activator of transcription 6",
  "term_label": "RNA polymerase II transcription regulator complex",
  "term_id": "GO:0090575",
  "gene_symbol": "STAT6",
  "gene": "UniProtKB:P42226"
}